{
  "gene": "UniProtKB:P01241",
  "gene_symbol": "GH1",
  "gene_name": "Somatotropin",
  "term_id": "GO:0046427",
  "term_label": "positive regulation of receptor signaling pathway via JAK-STAT"
}